{
  "gene_name": "3-hydroxyacyl-CoA dehydrogenase type-2",
  "gene": "UniProtKB:Q99714",
  "gene_symbol": "HSD17B10",
  "term_label": "mitochondrion",
  "term_id": "GO:0005739"
}